{
  "gene": "UniProtKB:Q6UXP3",
  "term_id": "GO:0031966",
  "gene_name": "Transmembrane protein 14EP",
  "term_label": "mitochondrial membrane",
  "gene_symbol": "TMEM14EP"
}